{
  "gene_symbol": "CEP128",
  "term_label": "spindle pole",
  "term_id": "GO:0000922",
  "gene_name": "Centrosomal protein of 128 kDa",
  "gene": "UniProtKB:Q6ZU80"
}